{
  "gene_symbol": "SLC35A2",
  "gene_name": "UDP-galactose translocator",
  "gene": "UniProtKB:P78381",
  "term_label": "Golgi membrane",
  "term_id": "GO:0000139"
}